{
  "term_label": "intracellular protein transport",
  "gene_name": "Syntaxin-1B",
  "gene_symbol": "STX1B",
  "gene": "UniProtKB:P61266",
  "term_id": "GO:0006886"
}